peptidyl-lysine modification to peptidyl-hypusine [GO:0008612] (biological process) Relationships: is a type of biosynthetic process [GO:0009058]; is a type of peptidyl-lysine modification [GO:0018205]; is a type of protein maturation [GO:0051604] Also known as: hypusine anabolism, hypusine anabolism from peptidyl-lysine, hypusine biosynthesis, hypusine biosynthetic process, hypusine biosynthetic process from peptidyl-lysine, hypusine formation, hypusine formation from peptidyl-lysine, hypusine synthesis, hypusine synthesis from peptidyl-lysine, hypusinylation, protein hypusination Definition: The modification of peptidyl-lysine to form hypusine, peptidyl-N6-(4-amino-2-hydroxybutyl)-L-lysine. Sources: GOC:ma, ISBN:0198547684, RESID:AA0116